{
  "term_id": "GO:0071896",
  "gene_symbol": "MPP7",
  "gene": "UniProtKB:Q5T2T1",
  "gene_name": "MAGUK p55 subfamily member 7",
  "term_label": "protein localization to adherens junction"
}